regulation of cell cycle G1/S phase transition [GO:1902806] (biological process) Subtypes: negative regulation of cell cycle G1/S phase transition [GO:1902807], positive regulation of cell cycle G1/S phase transition [GO:1902808], regulation of G1/S transition of mitotic cell cycle [GO:2000045] Sources: GOC:TermGenie, GOC:mtg_cell_cycle, GO_REF:0000058 Relationships: is a type of GO:1901987; regulates cell cycle G1/S phase transition [GO:0044843] Definition: Any signaling pathway that modulates the activity of a cell cycle cyclin-dependent protein kinase to modulate the switch from G1 phase to S phase of the cell cycle.